alphaV-beta3 integrin-CD47-FCER2 complex [GO:0071083] (cellular component) Also known as: ITGAV-ITGB3-CD447-FCER2 complex Relationships: is a type of plasma membrane protein complex [GO:0098797] References: PMID:10037797 Definition: A protein complex that consists of an alphaV-beta3 integrin complex bound to the cell surface protein CD47 and the low-affinity immunoglobulin epsilon Fc receptor (FCER2).